{
  "gene_name": "Probable ATP-dependent RNA helicase DDX41",
  "term_id": "UNKNOWN:0003",
  "gene_symbol": "DDX41",
  "gene": "UniProtKB:Q9UJV9",
  "term_label": "Unknown cellular component"
}